{
  "gene_name": "BTB_POZ domain-containing protein KCTD17",
  "term_label": "proteasome-mediated ubiquitin-dependent protein catabolic process",
  "gene_symbol": "KCTD17",
  "gene": "UniProtKB:Q8N5Z5",
  "term_id": "GO:0043161"
}